regulation of fibrinolysis [GO:0051917] (biological process) Subtypes: negative regulation of fibrinolysis [GO:0051918], positive regulation of fibrinolysis [GO:0051919] Definition: Any process that modulates the frequency, rate or extent of fibrinolysis, an ongoing process that solubilizes fibrin, resulting in the removal of small blood clots. Sources: GOC:ai Relationships: is a type of regulation of blood coagulation [GO:0030193]; regulates GO:0042730